{
  "gene_symbol": "TLR8",
  "term_id": "GO:0038187",
  "term_label": "pattern recognition receptor activity",
  "gene_name": "Toll-like receptor 8",
  "gene": "UniProtKB:Q9NR97"
}